inositol-5-diphosphate-1,2,3,4,6-pentakisphosphate diphosphatase activity [GO:0052845] (molecular function) Definition: Catalysis of the reaction: 5-diphospho-1D-myo-inositol 1,2,3,4,6-pentakisphosphate + H2O = 1D-myo-inositol 1,2,3,4,5,6-hexakisphosphate + phosphate + H+. References: PMID:10827188, PMID:11502751 Sources: RHEA:22384 Relationships: is a type of GO:0052842